{
  "gene_symbol": "GSG1L",
  "term_label": "Unknown molecular function",
  "gene_name": "Germ cell-specific gene 1-like protein",
  "term_id": "UNKNOWN:0001",
  "gene": "UniProtKB:Q6UXU4"
}